{
  "gene_name": "Sodium-dependent proline transporter",
  "term_id": "GO:1903804",
  "term_label": "glycine import across plasma membrane",
  "gene": "UniProtKB:Q99884",
  "gene_symbol": "SLC6A7"
}